{
  "term_id": "GO:0031783",
  "gene_symbol": "MRAP",
  "gene_name": "Melanocortin-2 receptor accessory protein",
  "term_label": "type 5 melanocortin receptor binding",
  "gene": "UniProtKB:Q8TCY5"
}